pristanoyl-CoA oxidase activity [GO:0016402] (molecular function) Relationships: is a type of GO:0003997 Sources: RHEA:40459 Definition: Catalysis of the reaction: (2S)-pristanoyl-CoA + O2 = (2E)-pristenoyl-CoA + H2O2.